{
  "gene_symbol": "SAMD15",
  "gene_name": "Sterile alpha motif domain-containing protein 15",
  "term_label": "protein serine/threonine kinase activator activity",
  "gene": "UniProtKB:Q9P1V8",
  "term_id": "GO:0043539"
}